chlorobenzene catabolic process [GO:0018914] (BP) Definition: The chemical reactions and pathways resulting in the breakdown of chlorobenzene, a derivative of benzene with a chlorine atoms attached to the ring. It is a colorless liquid that is manufactured for use as a solvent. It quickly evaporates in the air and is degraded by hydroxyl radicals that are produced photochemically. The gas acts as a source of ClOx, which helps in the breakdown of stratospheric ozone. References: PMID:10808489, PMID:8626733 Also known as: chlorobenzene metabolic process, chlorobenzene metabolism Relationships: is a type of catabolic process [GO:0009056]; is a type of GO:0042537; is a type of GO:0090345